(22S)-22-hydroxy-campest-4-en-3-one C-23 hydroxylase activity [GO:0102135] (molecular function) Sources: GOC:pz Relationships: is a type of oxidoreductase activity, acting on paired donors, with incorporation or reduction of molecular oxygen, NAD(P)H as one donor, and incorporation of one atom of oxygen [GO:0016709] Definition: Catalysis of the reaction: H+ + (22S)-22-hydroxycampest-4-en-3-one + NADPH + O2 = (22R,23R)-22,23-dihydroxy-campest-4-en-3-one + NADP + H2O.